exodeoxyribonuclease V complex [GO:0009338] (cellular component) Definition: An enzyme complex that catalyzes exonucleolytic cleavage (in the presence of ATP) in either 5' to 3' or 3' to 5' direction to yield 5'-phosphooligonucleotides. Exodeoxyribonuclease V shows a preference for double-stranded DNA and possesses DNA-dependent ATPase activity. It acts endonucleolytically on single-stranded circular DNA. References: PMID:1618858 Relationships: is a type of intracellular protein-containing complex [GO:0140535]; is a type of catalytic complex [GO:1902494]